{
  "gene": "UniProtKB:Q96PC2",
  "term_id": "GO:0000828",
  "gene_symbol": "IP6K3",
  "term_label": "inositol hexakisphosphate kinase activity",
  "gene_name": "Inositol hexakisphosphate kinase 3"
}